{
  "gene": "UniProtKB:Q99665",
  "term_label": "external side of plasma membrane",
  "term_id": "GO:0009897",
  "gene_name": "Interleukin-12 receptor subunit beta-2",
  "gene_symbol": "IL12RB2"
}